{
  "gene_symbol": "HRCT1",
  "term_id": "UNKNOWN:0001",
  "gene_name": "Histidine-rich carboxyl terminus protein 1",
  "term_label": "Unknown molecular function",
  "gene": "UniProtKB:Q6UXD1"
}